{
  "gene_symbol": "ACE",
  "term_id": "GO:0005615",
  "term_label": "extracellular space",
  "gene_name": "Angiotensin-converting enzyme",
  "gene": "UniProtKB:P12821"
}